{
  "gene": "UniProtKB:Q9UJT1",
  "term_id": "GO:0005200",
  "gene_name": "Tubulin delta chain",
  "gene_symbol": "TUBD1",
  "term_label": "structural constituent of cytoskeleton"
}